monoatomic cation:bicarbonate symporter activity [GO:0140410] (molecular function) Definition: Enables the transfer of a solute or solutes from one side of a membrane to the other according to the reaction: monoatomic cation(out) + HCO3-(out) = monoatomic cation(in) + HCO3-(in). References: PMID:27166256 Also known as: solute:bicarbonate symporter activity, monoatomic cation:hydrogencarbonate symporter activity Relationships: is a type of bicarbonate transmembrane transporter activity [GO:0015106]; is a type of solute:monoatomic cation symporter activity [GO:0015294] Subtypes: sodium:bicarbonate symporter activity [GO:0008510], zinc:bicarbonate symporter activity [GO:0140412]